{
  "term_id": "UNKNOWN:0002",
  "gene": "UniProtKB:Q96S95",
  "gene_symbol": "CAMK2N2",
  "term_label": "Unknown biological process",
  "gene_name": "Calcium_calmodulin-dependent protein kinase II inhibitor 2"
}